{
  "gene_name": "Insulinoma-associated protein 2",
  "gene_symbol": "INSM2",
  "gene": "UniProtKB:Q96T92",
  "term_label": "transcription repressor complex",
  "term_id": "GO:0017053"
}